{
  "gene": "UniProtKB:Q9NRZ9",
  "term_label": "DNA methylation-dependent constitutive heterochromatin formation",
  "term_id": "GO:0006346",
  "gene_symbol": "HELLS",
  "gene_name": "Lymphoid-specific helicase"
}